aerobic lactate catabolic process [GO:1990484] (BP) Definition: The chemical reactions and pathways resulting in the breakdown of lactate (2-hydroxypropanoic acid) in the presence of oxygen. Also known as: aerobic lactic acid catabolic process References: PMID:8941775 Sources: GOC:mengo_curators Relationships: is a type of lactate catabolic process [GO:1903457]